siderophore-dependent iron import pathway [GO:0180060] (biological process) Subtypes: siderophore-iron import into cell [GO:0033214], native siderophore export across plasma membrane [GO:0180061] Sources: GOC:vw Relationships: is a type of GO:0033212 Definition: A process in which iron siderophores (low-molecular-weight, high-affinity iron-chelating compounds) are exported to scavenge iron and the iron-loaded siderophores imported back into the cell by transmembrane transport or endocytosis.